positive regulation of gut granule assembly [GO:1904757] (biological process) Also known as: positive regulation of gut granule biogenesis, positive regulation of gut granule formation, up regulation of gut granule assembly, up regulation of gut granule biogenesis, up regulation of gut granule formation, up-regulation of gut granule assembly, up-regulation of gut granule biogenesis, up-regulation of gut granule formation, upregulation of gut granule assembly, upregulation of gut granule biogenesis, upregulation of gut granule formation, activation of gut granule assembly, activation of gut granule biogenesis, activation of gut granule formation Definition: Any process that activates or increases the frequency, rate or extent of gut granule assembly. Relationships: is_a positive regulation of organelle assembly [GO:1902117]; is a type of GO:1904755; positively regulates gut granule assembly [GO:1902900] References: PMID:17535251 Sources: GOC:TermGenie, GO_REF:0000058